{
  "gene": "UniProtKB:P61599",
  "gene_name": "N-alpha-acetyltransferase 20",
  "term_label": "NatB complex",
  "term_id": "GO:0031416",
  "gene_symbol": "NAA20"
}